{
  "term_id": "GO:0003743",
  "gene_name": "Eukaryotic translation initiation factor 5B",
  "term_label": "translation initiation factor activity",
  "gene": "UniProtKB:O60841",
  "gene_symbol": "EIF5B"
}